mitochondrial gene expression [GO:0140053] (biological process) Subtypes: mitochondrial RNA processing [GO:0000963] Definition: The process in which a mitochondrial gene's sequence is converted into a mature gene product or products (proteins or RNA). This includes the production of an RNA transcript as well as any processing to produce a mature RNA product or an mRNA or circRNA (for protein-coding genes) and the translation of that mRNA or circRNA into protein. Protein maturation is included when required to form an active form of a product from an inactive precursor form. Regulation: regulated by regulation of mitochondrial gene expression [GO:0062125] References: PMID:27058308 Relationships: is_a gene expression [GO:0010467]; occurs in mitochondrion [GO:0005739]